{
  "term_id": "GO:0006954",
  "gene_symbol": "IL18",
  "term_label": "inflammatory response",
  "gene_name": "Interleukin-18",
  "gene": "UniProtKB:Q14116"
}